{
  "gene": "UniProtKB:A0A1W2PQ73",
  "term_id": "GO:0005634",
  "gene_name": "ETS domain-containing transcription factor ERF-like",
  "gene_symbol": "ERFL",
  "term_label": "nucleus"
}